{
  "gene_symbol": "APOA4",
  "term_label": "cholesterol metabolic process",
  "gene_name": "Apolipoprotein A-IV",
  "gene": "UniProtKB:P06727",
  "term_id": "GO:0008203"
}